{
  "gene_symbol": "AIRE",
  "term_id": "GO:0045944",
  "gene_name": "Autoimmune regulator",
  "term_label": "positive regulation of transcription by RNA polymerase II",
  "gene": "UniProtKB:O43918"
}